neuron projection extension [GO:1990138] (biological process) Relationships: is a type of developmental cell growth [GO:0048588]; is a type of developmental growth involved in morphogenesis [GO:0060560]; is part of neuron projection morphogenesis [GO:0048812] Also known as: neuron process extension, neuron protrusion extension, neuronal cell projection extension, neurite extension Subtypes: axon extension [GO:0048675], dendrite extension [GO:0097484], sympathetic neuron projection extension [GO:0097490], neuron projection extension involved in neuron projection guidance [GO:1902284] Definition: Long distance growth of a single neuron projection involved in cellular development. A neuron projection is a prolongation or process extending from a nerve cell, e.g. an axon or dendrite. References: PMID:22790009 Sources: GOC:BHF, GOC:rl